{
  "gene": "UniProtKB:Q9H741",
  "gene_name": "SREBP regulating gene protein",
  "term_id": "UNKNOWN:0001",
  "gene_symbol": "SPRING1",
  "term_label": "Unknown molecular function"
}